{
  "term_label": "plasma membrane",
  "gene_name": "Probable G-protein coupled receptor 25",
  "gene_symbol": "GPR25",
  "gene": "UniProtKB:O00155",
  "term_id": "GO:0005886"
}